{
  "term_label": "Unknown biological process",
  "gene": "UniProtKB:Q5VU36",
  "gene_symbol": "SPATA31A5",
  "term_id": "UNKNOWN:0002",
  "gene_name": "Spermatogenesis-associated protein 31A5"
}